{
  "term_label": "Unknown cellular component",
  "gene_name": "cAMP-specific 3',5'-cyclic phosphodiesterase 4A",
  "term_id": "UNKNOWN:0003",
  "gene": "UniProtKB:P27815",
  "gene_symbol": "PDE4A"
}